{
  "gene": "UniProtKB:Q71DI3",
  "term_label": "nucleosome",
  "term_id": "GO:0000786",
  "gene_symbol": "H3C13",
  "gene_name": "Histone H3.2"
}